{
  "gene_symbol": "PLCXD1",
  "gene_name": "PI-PLC X domain-containing protein 1",
  "term_id": "UNKNOWN:0003",
  "gene": "UniProtKB:Q9NUJ7",
  "term_label": "Unknown cellular component"
}